U4atac snRNA binding [GO:0030622] (molecular function) Definition: Binding to a U4atac small nuclear RNA (U4atac snRNA). Sources: GOC:jl Relationships: is a type of snRNA binding [GO:0017069]